{
  "term_id": "GO:0098609",
  "term_label": "cell-cell adhesion",
  "gene": "UniProtKB:Q13683",
  "gene_symbol": "ITGA7",
  "gene_name": "Integrin alpha-7"
}